transcription coregulator binding [GO:0001221] (molecular function) Definition: Binding to a transcription coregulator, a protein involved in regulation of transcription via protein-protein interactions with transcription factors and other transcription regulatory proteins. Cofactors do not bind DNA directly, but rather mediate protein-protein interactions between regulatory transcription factors and the basal transcription machinery. Subtypes: transcription corepressor binding [GO:0001222], transcription coactivator binding [GO:0001223] Relationships: is_a transcription factor binding [GO:0008134] Sources: GOC:krc Also known as: RNA polymerase II transcription cofactor binding, RNA polymerase II transcription coregulator binding, transcription cofactor binding